{
  "gene": "UniProtKB:O75506",
  "term_id": "GO:0070370",
  "term_label": "cellular heat acclimation",
  "gene_name": "Heat shock factor-binding protein 1",
  "gene_symbol": "HSBP1"
}